{
  "gene_name": "Vascular endothelial growth factor A, long form",
  "term_id": "GO:0001666",
  "term_label": "response to hypoxia",
  "gene_symbol": "VEGFA",
  "gene": "UniProtKB:P15692"
}